pentose transmembrane transport [GO:0015750] (biological process) Definition: The process in which pentose is transported across a lipid bilayer, from one side of a membrane to the other. A pentose is any aldose with a chain of five carbon atoms in the molecule. Sources: GOC:ai Also known as: pentose transport Relationships: is a type of monosaccharide transmembrane transport [GO:0015749] Subtypes: arabinose transmembrane transport [GO:0015751], D-ribose transmembrane transport [GO:0015752], D-xylose transmembrane transport [GO:0015753]